{
  "term_id": "GO:0000978",
  "term_label": "RNA polymerase II cis-regulatory region sequence-specific DNA binding",
  "gene_symbol": "DLX4",
  "gene_name": "Homeobox protein DLX-4",
  "gene": "UniProtKB:Q92988"
}